{
  "gene_symbol": "KCNK17",
  "term_label": "outward rectifier potassium channel activity",
  "gene": "UniProtKB:Q96T54",
  "term_id": "GO:0015271",
  "gene_name": "Potassium channel subfamily K member 17"
}